neuroendocrine cell differentiation involved in prostate gland acinus development [GO:0060531] (biological process) Relationships: is_a epithelial cell differentiation involved in prostate gland development [GO:0060742]; is a type of neuroendocrine cell differentiation [GO:0061101]; is part of prostate glandular acinus development [GO:0060525] Definition: The process in which relatively unspecialized cells acquires specialized structural and functions of a neuroendocrine cell of the prostate gland acinus. References: PMID:18977204 Sources: GOC:dph